{
  "term_id": "GO:0015485",
  "term_label": "cholesterol binding",
  "gene_name": "StAR-related lipid transfer protein 4",
  "gene": "UniProtKB:Q96DR4",
  "gene_symbol": "STARD4"
}